procollagen-proline dioxygenase activity [GO:0019798] (molecular function) Definition: Catalysis of the reaction: procollagen L-proline + 2-oxoglutarate + O2 = procollagen trans-hydroxy-L-proline + succinate + CO2. Subtypes: GO:0004656, procollagen-proline 3-dioxygenase activity [GO:0019797] Relationships: is a type of peptidyl-proline dioxygenase activity [GO:0031543] References: PMID:4371784 Sources: GOC:mah